regulation of calcium ion transmembrane transport [GO:1903169] (biological process) Note: human HRC regulates RYR2 and thus regulates transmembrane transport of calcium from SR to cytosol Relationships: is a type of regulation of calcium ion transport [GO:0051924]; is a type of GO:1904062; regulates GO:0070588 Definition: Any process that modulates the frequency, rate or extent of calcium ion transmembrane transport. Also known as: regulation of calcium ion membrane transport, regulation of transmembrane calcium transport Subtypes: GO:0010522, regulation of release of sequestered calcium ion into cytosol [GO:0051279], regulation of calcium import into the mitochondrion [GO:0110097], regulation of calcium ion transmembrane transport via high voltage-gated calcium channel [GO:1902514], negative regulation of calcium ion transmembrane transport [GO:1903170], positive regulation of calcium ion transmembrane transport [GO:1904427], regulation of calcium ion import across plasma membrane [GO:1905664], regulation of calcium ion export across plasma membrane [GO:1905912] References: PMID:24125847 Sources: GOC:BHF, GOC:TermGenie, GOC:rl, GO_REF:0000058